{
  "term_id": "GO:0030674",
  "term_label": "protein-macromolecule adaptor activity",
  "gene": "UniProtKB:O94875",
  "gene_name": "Sorbin and SH3 domain-containing protein 2",
  "gene_symbol": "SORBS2"
}